{
  "gene": "UniProtKB:O95715",
  "term_id": "UNKNOWN:0001",
  "gene_symbol": "CXCL14",
  "gene_name": "C-X-C motif chemokine 14",
  "term_label": "Unknown molecular function"
}